{
  "term_label": "Unknown biological process",
  "gene": "UniProtKB:A0A0A0MT86",
  "gene_symbol": "IGLJ5",
  "term_id": "UNKNOWN:0002",
  "gene_name": "Immunoglobulin lambda joining 5 (non-functional) (Fragment)"
}